{
  "term_label": "tRNA methylation",
  "gene": "UniProtKB:Q9BVS5",
  "gene_name": "tRNA (adenine(58)-N(1))-methyltransferase, mitochondrial",
  "term_id": "GO:0030488",
  "gene_symbol": "TRMT61B"
}